{
  "gene": "UniProtKB:Q13241",
  "gene_symbol": "KLRD1",
  "term_label": "HLA-E specific inhibitory MHC class Ib receptor activity",
  "gene_name": "Natural killer cells antigen CD94",
  "term_id": "GO:0062082"
}